B cell tolerance induction [GO:0002514] (biological process) Subtypes: GO:0002451, central B cell tolerance induction [GO:0002510], B cell anergy [GO:0002515] References: PMID:16460922 Sources: GOC:jal, ISBN:0781735149 Regulation: regulated by GO:0002661; negatively regulated by negative regulation of B cell tolerance induction [GO:0002662]; RO_0002213 by positive regulation of B cell tolerance induction [GO:0002663] Also known as: B lymphocyte tolerance induction, B-cell tolerance induction, B-lymphocyte tolerance induction Relationships: is_a GO:0002507 Definition: A process involving any mechanism for tolerance induction in B cells.